{
  "gene_name": "Serine_threonine-protein kinase ULK3",
  "term_id": "GO:0010506",
  "term_label": "regulation of autophagy",
  "gene_symbol": "ULK3",
  "gene": "UniProtKB:Q6PHR2"
}